{
  "term_id": "UNKNOWN:0001",
  "gene_symbol": "C1orf140",
  "gene_name": "Putative uncharacterized protein C1orf140",
  "gene": "UniProtKB:Q5VVS0",
  "term_label": "Unknown molecular function"
}